{
  "gene": "UniProtKB:P49281",
  "gene_name": "Natural resistance-associated macrophage protein 2",
  "term_label": "intracellular manganese ion homeostasis",
  "term_id": "GO:0030026",
  "gene_symbol": "SLC11A2"
}